activation of store-operated calcium channel activity [GO:0032237] (biological process) Relationships: is_a positive regulation of store-operated calcium channel activity [GO:1901341] Sources: GOC:mah Definition: A process that initiates the activity of an inactive store-operated calcium channel.